{
  "term_label": "membrane",
  "term_id": "GO:0016020",
  "gene_name": "ATP-dependent 6-phosphofructokinase, muscle type",
  "gene_symbol": "PFKM",
  "gene": "UniProtKB:P08237"
}